futile creatine cycle [GO:0140651] (biological process) References: PMID:33597756, PMID:33981039 Relationships: is a type of GO:0008152; is part of adaptive thermogenesis [GO:1990845]; has part creatine kinase activity [GO:0004111]; has part GO:0050187 Definition: The phosphorylation and dephosphorylation of creatine in a futile cycle, which dissipates the high energy charge of phosphocreatine as heat without performing any mechanical or chemical work. The futile creatine cycle takes place in thermogenic fat cells and is part of adaptive thermogenesis.